{
  "term_label": "Unknown biological process",
  "gene": "UniProtKB:Q8NEB7",
  "term_id": "UNKNOWN:0002",
  "gene_name": "Acrosin-binding protein",
  "gene_symbol": "ACRBP"
}